metanephric epithelium development [GO:0072207] (biological process) Definition: The process whose specific outcome is the progression of an epithelium in the metanephros over time, from its formation to the mature structure. An epithelium is a tissue that covers the internal or external surfaces of an anatomical structure. Subtypes: metanephric tubule development [GO:0072170], metanephric nephron epithelium development [GO:0072243] Sources: GOC:mtg_kidney_jan10 Relationships: is_a kidney epithelium development [GO:0072073]; is part of metanephros development [GO:0001656]